regulation of cell chemotaxis to fibroblast growth factor [GO:1904847] (biological process) References: PMID:23233752 Sources: GOC:BHF, GOC:BHF_miRNA, GOC:TermGenie, GOC:rph, GO_REF:0000058 Definition: Any process that modulates the frequency, rate or extent of cell chemotaxis to fibroblast growth factor. Relationships: is a type of regulation of cell migration [GO:0030334]; is a type of regulation of chemotaxis [GO:0050920]; is_a regulation of cellular response to growth factor stimulus [GO:0090287]; regulates GO:0035766 Subtypes: negative regulation of cell chemotaxis to fibroblast growth factor [GO:1904848], positive regulation of cell chemotaxis to fibroblast growth factor [GO:1904849], regulation of endothelial cell chemotaxis to fibroblast growth factor [GO:2000544]